negative regulation of elastin catabolic process [GO:0060311] (BP) Definition: Any process that decreases the rate, frequency or extent of elastin catabolism, the chemical reactions and pathways resulting in the breakdown of elastin. Sources: GOC:BHF, GOC:dph, GOC:tb Relationships: is a type of negative regulation of protein catabolic process [GO:0042177]; is_a regulation of elastin catabolic process [GO:0060310]; is a type of negative regulation of glycoprotein metabolic process [GO:1903019]; negatively regulates elastin catabolic process [GO:0060309] Also known as: down-regulation of elastin catabolic process, negative regulation of elastin breakdown, negative regulation of elastin catabolism, negative regulation of elastin degradation